glutamate synthase complex (NADH) [GO:0031027] (cellular component) Definition: A protein complex that in yeast consists of a large and a small subunit. Possesses glutamate synthase (NADH) activity. References: PMID:7047525 Sources: GOC:jl Relationships: is a type of glutamate synthase complex [GO:0031026] Subtypes: mitochondrial glutamate synthase complex (NADH) [GO:0043294]